{
  "gene": "UniProtKB:Q13075",
  "term_label": "pyroptotic inflammatory response",
  "term_id": "GO:0070269",
  "gene_name": "Baculoviral IAP repeat-containing protein 1",
  "gene_symbol": "NAIP"
}